contractile muscle fiber [GO:0043292] (cellular component) Definition: Fibers, composed of actin, myosin, and associated proteins, found in cells of smooth or striated muscle. Also known as: contractile fibre Subtypes: myofibril [GO:0030016], smooth muscle contractile fiber [GO:0030485] Sources: GOC:go_curators, ISBN:0815316194 Relationships: is a type of intracellular membraneless organelle [GO:0043232]; is a type of supramolecular fiber [GO:0099512]; is part of cytoplasm [GO:0005737]